{
  "term_id": "GO:0006457",
  "term_label": "protein folding",
  "gene_symbol": "HSP90AB1",
  "gene": "UniProtKB:P08238",
  "gene_name": "Heat shock protein HSP 90-beta"
}